{
  "gene_symbol": "AQP12A",
  "gene_name": "Aquaporin-12A",
  "term_label": "cytoplasm",
  "term_id": "GO:0005737",
  "gene": "UniProtKB:Q8IXF9"
}